{
  "term_label": "mRNA 3'-UTR binding",
  "gene": "UniProtKB:Q96PM9",
  "gene_symbol": "ZNF385A",
  "gene_name": "Zinc finger protein 385A",
  "term_id": "GO:0003730"
}